{
  "term_label": "RNA polymerase II cis-regulatory region sequence-specific DNA binding",
  "gene_symbol": "MLXIP",
  "term_id": "GO:0000978",
  "gene_name": "MLX-interacting protein",
  "gene": "UniProtKB:Q9HAP2"
}